positive regulation of cellular response to oxidative stress [GO:1900409] (biological process) Definition: Any process that activates or increases the frequency, rate or extent of cellular response to oxidative stress. Relationships: is a type of positive regulation of cellular process [GO:0048522]; is a type of GO:1900407; is a type of positive regulation of response to oxidative stress [GO:1902884]; positively regulates GO:0034599 Sources: GOC:TermGenie, GOC:mah Also known as: up regulation of cellular response to oxidative stress, up-regulation of cellular response to oxidative stress, upregulation of cellular response to oxidative stress, activation of adaptive response to oxidative stress, activation of cellular response to oxidative stress, positive regulation of adaptive response to oxidative stress, up regulation of adaptive response to oxidative stress, up-regulation of adaptive response to oxidative stress, upregulation of adaptive response to oxidative stress